{
  "term_label": "extracellular space",
  "gene": "UniProtKB:P49763",
  "term_id": "GO:0005615",
  "gene_name": "Placenta growth factor",
  "gene_symbol": "PGF"
}